{
  "gene": "UniProtKB:P16157",
  "term_label": "spectrin binding",
  "gene_symbol": "ANK1",
  "term_id": "GO:0030507",
  "gene_name": "Ankyrin-1"
}